arabinose-5-phosphate isomerase activity [GO:0019146] (molecular function) Definition: Catalysis of the reaction: D-arabinose 5-phosphate = D-ribulose 5-phosphate + 2 H+. Sources: EC:5.3.1.13, RHEA:23104 Also known as: D-arabinose-5-phosphate aldose-ketose-isomerase activity, D-arabinose-5-phosphate ketol-isomerase activity, arabinose phosphate isomerase activity, phosphoarabinoisomerase activity Relationships: is a type of intramolecular oxidoreductase activity, interconverting aldoses and ketoses [GO:0016861]